{
  "gene_symbol": "CBX2",
  "gene_name": "Chromobox protein homolog 2",
  "gene": "UniProtKB:Q14781",
  "term_label": "PRC1 complex",
  "term_id": "GO:0035102"
}